regulation of corticosteroid hormone secretion [GO:2000846] (biological process) Sources: GOC:sl Relationships: is a type of regulation of steroid hormone secretion [GO:2000831]; regulates corticosteroid hormone secretion [GO:0035930] Definition: Any process that modulates the frequency, rate or extent of corticosteroid hormone secretion. Also known as: regulation of corticosteroid secretion Subtypes: GO:2000847, positive regulation of corticosteroid hormone secretion [GO:2000848], regulation of glucocorticoid secretion [GO:2000849], regulation of mineralocorticoid secretion [GO:2000855]